ciliary pocket [GO:0020016] (cellular component) Sources: GOC:cilia, GOC:mb Definition: Invagination of the plasma membrane from which a cilium (also called flagellum) protrudes. Note: Note that cilia and eukaryotic flagella are deemed to be equivalent. In this case community usage is mostly 'flagellar', but the primary term name reflects the cilium parentage. Also known as: cilial pocket, cilium pocket, flagellar pocket Relationships: is_a cellular anatomical structure [GO:0110165]; is part of cilium [GO:0005929]